{
  "gene": "UniProtKB:P49006",
  "term_label": "actin filament binding",
  "term_id": "GO:0051015",
  "gene_symbol": "MARCKSL1",
  "gene_name": "MARCKS-related protein"
}